{
  "gene": "UniProtKB:Q8ND04",
  "gene_symbol": "SMG8",
  "term_label": "nuclear-transcribed mRNA catabolic process, nonsense-mediated decay",
  "gene_name": "Nonsense-mediated mRNA decay factor SMG8",
  "term_id": "GO:0000184"
}